{
  "gene": "UniProtKB:Q8NBJ9",
  "term_id": "GO:0005764",
  "gene_name": "SID1 transmembrane family member 2",
  "gene_symbol": "SIDT2",
  "term_label": "lysosome"
}